{
  "term_label": "mitotic recombination",
  "term_id": "GO:0006312",
  "gene": "UniProtKB:Q14565",
  "gene_name": "Meiotic recombination protein DMC1_LIM15 homolog",
  "gene_symbol": "DMC1"
}